positive regulation of endosomal vesicle fusion [GO:1905363] (BP) Also known as: positive regulation of endosome vesicle fusion, up regulation of endosomal vesicle fusion, up regulation of endosome vesicle fusion, up-regulation of endosomal vesicle fusion, up-regulation of endosome vesicle fusion, upregulation of endosomal vesicle fusion, upregulation of endosome vesicle fusion, activation of endosomal vesicle fusion, activation of endosome vesicle fusion References: PMID:26911690 Sources: GOC:PARL, GOC:TermGenie, GOC:bc, GO_REF:0000058 Definition: Any process that activates or increases the frequency, rate or extent of endosomal vesicle fusion. Relationships: is_a positive regulation of vesicle fusion [GO:0031340]; is_a regulation of endosomal vesicle fusion [GO:1905364]; positively regulates endosomal vesicle fusion [GO:0034058]